{
  "term_label": "misfolded protein binding",
  "term_id": "GO:0051787",
  "gene": "UniProtKB:Q13217",
  "gene_symbol": "DNAJC3",
  "gene_name": "DnaJ homolog subfamily C member 3"
}